{
  "gene": "UniProtKB:Q9UPS6",
  "gene_name": "Histone-lysine N-methyltransferase SETD1B",
  "gene_symbol": "SETD1B",
  "term_id": "UNKNOWN:0001",
  "term_label": "Unknown molecular function"
}